{
  "gene_name": "NADH dehydrogenase [ubiquinone] 1 beta subcomplex subunit 6",
  "gene_symbol": "NDUFB6",
  "gene": "UniProtKB:O95139",
  "term_id": "GO:0042775",
  "term_label": "mitochondrial ATP synthesis coupled electron transport"
}